ATPase coupled ion transmembrane transporter activity involved in regulation of postsynaptic membrane potential [GO:0099581] (molecular function) Definition: Any ATPase coupled ion transmembrane transporter activity, occurring in the postsynaptic membrane, that is involved in regulation of postsynaptic membrane potential. Sources: GOC:dos Also known as: ATPase coupled ion transmembrane transporter activity involved in regulation of post-synaptic membrane potential, ATPase-coupled ion transmembrane transporter activity involved in regulation of postsynaptic membrane potential Relationships: is a type of GO:0042625; is part of regulation of postsynaptic membrane potential [GO:0060078]; occurs in postsynaptic membrane [GO:0045211]